{
  "gene_symbol": "ZNF416",
  "gene_name": "Zinc finger protein 416",
  "term_id": "GO:0005634",
  "gene": "UniProtKB:Q9BWM5",
  "term_label": "nucleus"
}